{
  "gene": "UniProtKB:P51800",
  "gene_name": "Chloride channel protein ClC-Ka",
  "term_label": "chloride transport",
  "term_id": "GO:0006821",
  "gene_symbol": "CLCNKA"
}